{
  "term_label": "kinocilium",
  "gene_name": "Glutaredoxin domain-containing cysteine-rich protein 1",
  "term_id": "GO:0060091",
  "gene_symbol": "GRXCR1",
  "gene": "UniProtKB:A8MXD5"
}